{
  "term_id": "GO:0003714",
  "gene_symbol": "MIER3",
  "gene_name": "Mesoderm induction early response protein 3",
  "term_label": "transcription corepressor activity",
  "gene": "UniProtKB:Q7Z3K6"
}